{
  "gene": "UniProtKB:P16383",
  "term_label": "mRNA splicing, via spliceosome",
  "gene_name": "Intron Large complex component GCFC2",
  "gene_symbol": "GCFC2",
  "term_id": "GO:0000398"
}